regulation of fibroblast chemotaxis [GO:1905210] (biological process) Definition: Any process that modulates the frequency, rate or extent of fibroblast chemotaxis. References: PMID:8760137 Sources: GOC:TermGenie, GO_REF:0000058 Relationships: is a type of regulation of cell migration [GO:0030334]; is a type of regulation of chemotaxis [GO:0050920]; regulates GO:1990956 Subtypes: negative regulation of fibroblast chemotaxis [GO:1905211], positive regulation of fibroblast chemotaxis [GO:1905212]